rRNA (guanine-N7-)-methyltransferase activity [GO:0070043] (molecular function) Definition: Catalysis of the reaction: S-adenosyl-L-methionine + rRNA = S-adenosyl-L-homocysteine + rRNA containing N7-methylguanine. Sources: GOC:imk, GOC:mah Relationships: is a type of GO:0008170; is a type of rRNA (guanine) methyltransferase activity [GO:0016435]; is part of rRNA (guanine-N7)-methylation [GO:0070476]